{
  "gene": "UniProtKB:P78395",
  "term_id": "GO:1990756",
  "term_label": "ubiquitin-like ligase-substrate adaptor activity",
  "gene_symbol": "PRAME",
  "gene_name": "Melanoma antigen preferentially expressed in tumors"
}